{
  "term_label": "integrin binding",
  "gene_symbol": "ITGB3",
  "term_id": "GO:0005178",
  "gene": "UniProtKB:P05106",
  "gene_name": "Integrin beta-3"
}